{
  "gene_name": "Myosin regulatory light chain 12B",
  "term_label": "Unknown biological process",
  "gene_symbol": "MYL12B",
  "gene": "UniProtKB:O14950",
  "term_id": "UNKNOWN:0002"
}